{
  "gene": "UniProtKB:Q13813",
  "term_id": "GO:0005886",
  "gene_symbol": "SPTAN1",
  "term_label": "plasma membrane",
  "gene_name": "Spectrin alpha chain, non-erythrocytic 1"
}